{
  "gene": "UniProtKB:P43632",
  "term_label": "plasma membrane",
  "term_id": "GO:0005886",
  "gene_symbol": "KIR2DS4",
  "gene_name": "Killer cell immunoglobulin-like receptor 2DS4"
}